regulation of 3'-UTR-mediated mRNA stabilization [GO:1905868] (biological process) Subtypes: negative regulation of 3'-UTR-mediated mRNA stabilization [GO:1905869], positive regulation of 3'-UTR-mediated mRNA stabilization [GO:1905870] Relationships: is_a regulation of mRNA stability [GO:0043488]; regulates 3'-UTR-mediated mRNA stabilization [GO:0070935] References: PMID:19737525 Sources: GOC:TermGenie, GO_REF:0000058 Definition: Any process that modulates the frequency, rate or extent of 3'-UTR-mediated mRNA stabilization. Also known as: regulation of 3'-untranslated region-mediated mRNA stabilization